regulation of gastric acid secretion [GO:0060453] (biological process) Relationships: is a type of regulation of digestive system process [GO:0044058]; is a type of regulation of secretion [GO:0051046]; regulates GO:0001696 Sources: GOC:dph, GOC:tb Definition: Any process that modulates the rate frequency or extent of gastric secretion. Gastric secretion is the regulated release of gastric acid (hydrochloric acid) by parietal or oxyntic cells during digestion. Subtypes: GO:0060454, negative regulation of gastric acid secretion [GO:0060455], GO:1903639